COP9 signalosome [GO:0008180] (cellular component) Definition: A protein complex that catalyzes the deneddylation of proteins, including the cullin component of SCF ubiquitin E3 ligase; deneddylation increases the activity of cullin family ubiquitin ligases. The signalosome is involved in many regulatory process, including some which control development, in many species; also regulates photomorphogenesis in plants; in many species its subunits are highly similar to those of the proteasome. References: PMID:11019806, PMID:12186635, PMID:14570571 Also known as: signalosome, COP9 complex, CSN Relationships: is a type of GO:0140513